{
  "gene_symbol": "ARGLU1",
  "term_label": "Unknown biological process",
  "gene_name": "Arginine and glutamate-rich protein 1",
  "gene": "UniProtKB:Q9NWB6",
  "term_id": "UNKNOWN:0002"
}